{
  "gene_name": "FYVE and coiled-coil domain-containing protein 1",
  "gene": "UniProtKB:Q9BQS8",
  "term_label": "Unknown molecular function",
  "term_id": "UNKNOWN:0001",
  "gene_symbol": "FYCO1"
}